central element [GO:0000801] (cellular component) Sources: GOC:elh Relationships: is a type of cellular anatomical structure [GO:0110165]; is part of synaptonemal complex [GO:0000795] Definition: A structural unit of the synaptonemal complex found between the lateral elements.